{
  "term_label": "cytoplasm",
  "term_id": "GO:0005737",
  "gene_name": "Rho GTPase-activating protein 39",
  "gene": "UniProtKB:Q9C0H5",
  "gene_symbol": "ARHGAP39"
}